positive regulation of L-glutamate import across plasma membrane [GO:0002038] (biological process) Also known as: positive regulation of L-glutamate import, positive regulation of L-glutamate transport, up regulation of L-glutamate transport, upregulation of L-glutamate transport, up regulation of L-glutamate import, up-regulation of L-glutamate import, up-regulation of L-glutamate transport, upregulation of L-glutamate import, activation of L-glutamate import, activation of L-glutamate transport, activation of L-glutamate uptake, stimulation of L-glutamate transport, positive regulation of L-glutamate uptake, up regulation of L-glutamate uptake, up-regulation of L-glutamate uptake, upregulation of L-glutamate uptake Sources: GOC:TermGenie Definition: Any process that activates or increases the frequency, rate or extent of L-glutamate import into a cell. Relationships: is a type of GO:0002036; is a type of positive regulation of organic acid transport [GO:0032892]; is a type of GO:0034764; is a type of positive regulation of amino acid transport [GO:0051957]; positively regulates L-glutamate import across plasma membrane [GO:0098712] Subtypes: positive regulation of glutamate uptake involved in transmission of nerve impulse [GO:0051951]